melanin-concentrating hormone receptor activity [GO:0030273] (molecular function) Sources: GOC:mah Also known as: MCH receptor Definition: Combining with the cyclic peptide hormone melanin-concentrating hormone to initiate a change in cell activity. Relationships: is a type of G protein-coupled receptor activity [GO:0004930]; is a type of GO:0016500